{
  "gene_name": "Neutrophil collagenase",
  "gene": "UniProtKB:P22894",
  "gene_symbol": "MMP8",
  "term_label": "Unknown cellular component",
  "term_id": "UNKNOWN:0003"
}